{
  "gene_name": "E3 ubiquitin-protein ligase Praja-2",
  "term_label": "cytoplasm",
  "term_id": "GO:0005737",
  "gene_symbol": "PJA2",
  "gene": "UniProtKB:O43164"
}